{
  "gene": "UniProtKB:Q15573",
  "term_id": "UNKNOWN:0003",
  "gene_name": "TATA box-binding protein-associated factor RNA polymerase I subunit A",
  "gene_symbol": "TAF1A",
  "term_label": "Unknown cellular component"
}